4-coumarate-CoA ligase activity [GO:0016207] (molecular function) Relationships: is a type of CoA-ligase activity [GO:0016405]; is a type of GO:0016878 Also known as: 4-coumarate-CoA synthetase activity, 4-coumarate:CoA ligase activity, 4-coumarate:CoA ligase (AMP-forming), 4-coumarate:coenzyme A ligase activity, 4-coumaroyl-CoA synthase activity, 4-coumaroyl-CoA synthetase activity, 4-coumaryl-CoA synthetase activity, 4CL, caffeolyl coenzyme A synthetase activity, feruloyl CoA ligase activity, feruloyl coenzyme A synthetase activity, hydroxycinnamate:CoA ligase activity, hydroxycinnamoyl CoA synthetase activity, p-coumaroyl CoA ligase activity, p-coumaryl coenzyme A synthetase activity, p-coumaryl-CoA ligase activity, p-coumaryl-CoA synthetase activity, p-hydroxycinnamic acid:CoA ligase activity, p-hydroxycinnamoyl coenzyme A synthetase activity, sinapoyl coenzyme A synthetase activity Definition: Catalysis of the reaction: ATP + 4-coumarate + CoA = AMP + diphosphate + 4-coumaroyl-CoA. Sources: EC:6.2.1.12